{
  "gene": "UniProtKB:D6RCP7",
  "gene_name": "Ubiquitin carboxyl-terminal hydrolase 17-like protein 19",
  "gene_symbol": "USP17L19",
  "term_id": "GO:0005634",
  "term_label": "nucleus"
}